{
  "gene_name": "Protocadherin gamma-B3",
  "term_label": "plasma membrane",
  "gene_symbol": "PCDHGB3",
  "gene": "UniProtKB:Q9Y5G1",
  "term_id": "GO:0005886"
}